{
  "gene_name": "Putative uncharacterized protein C8orf44",
  "term_id": "UNKNOWN:0002",
  "gene_symbol": "C8orf44",
  "term_label": "Unknown biological process",
  "gene": "UniProtKB:Q96CB5"
}